embryonic body morphogenesis [GO:0010172] (biological process) Sources: GOC:ems Definition: The process in which the anatomical structures of the embryonic soma are generated and organized. Relationships: is a type of body morphogenesis [GO:0010171]; is a type of embryonic morphogenesis [GO:0048598]